{
  "term_label": "skeletal system development",
  "term_id": "GO:0001501",
  "gene": "UniProtKB:Q86UW8",
  "gene_symbol": "HAPLN4",
  "gene_name": "Hyaluronan and proteoglycan link protein 4"
}